forked DNA-dependent helicase activity [GO:0061749] (molecular function) Definition: Unwinding a DNA helix containing forked DNA, driven by ATP hydrolysis. References: PMID:26277776 Sources: GOC:dph Relationships: is a type of DNA helicase activity [GO:0003678]